{
  "gene": "UniProtKB:Q15363",
  "gene_symbol": "TMED2",
  "gene_name": "Transmembrane emp24 domain-containing protein 2",
  "term_id": "UNKNOWN:0001",
  "term_label": "Unknown molecular function"
}